{
  "gene_name": "Elongation of very long chain fatty acids protein 6",
  "gene_symbol": "ELOVL6",
  "term_id": "GO:0034625",
  "term_label": "fatty acid elongation, monounsaturated fatty acid",
  "gene": "UniProtKB:Q9H5J4"
}